protein-glutamate methylesterase activity [GO:0008984] (molecular function) Sources: EC:3.1.1.61, RESID:AA0072 Relationships: is a type of GO:0051723 Definition: Catalysis of the reaction: protein L-glutamate O(5)-methyl ester + H2O = protein L-glutamate + methanol. Also known as: CheB methylesterase activity, chemotaxis-specific methylesterase activity, methyl-accepting chemotaxis protein methyl-esterase activity, methylesterase CheB activity, protein-L-glutamate-5-O-methyl-ester acylhydrolase activity, protein-L-glutamate-O5-methyl-ester acylhydrolase activity